B cell receptor editing [GO:0002452] (biological process) Definition: The process of replacing receptors on B cells, in which RAG gene expression allows continued light-chain gene rearrangement and expression of a new light change which combines with the previous heavy chain to form a new receptor. Also known as: B lymphocyte receptor editing, B-cell receptor editing, B-lymphocyte receptor editing Relationships: is a type of somatic recombination of immunoglobulin gene segments [GO:0016447] Sources: GOC:jal, ISBN:0781735149 Subtypes: GO:0002345, central B cell receptor editing [GO:0002511]